{
  "gene_name": "Oligodendrocyte transcription factor 1",
  "gene": "UniProtKB:Q8TAK6",
  "gene_symbol": "OLIG1",
  "term_id": "GO:0007423",
  "term_label": "sensory organ development"
}